telomeric repeat-containing RNA binding [GO:0061752] (molecular function) Definition: Binding to long non-coding RNA molecules transcribed from subtelomeric regions in most eukaryotes. Telomeric repeat-containing RNA (TERRA) molecules consist of subtelomeric-derived sequences and G-rich telomeric repeats. References: PMID:20655916 Sources: GOC:BHF, GOC:BHF_telomere, GOC:dph, GOC:jbu Also known as: TERRA binding Relationships: is a type of RNA binding [GO:0003723]